Purkinje myocyte to ventricular cardiac muscle cell communication [GO:0086068] (biological process) Definition: The process that mediates interactions between a Purkinje myocyte and its surroundings that contributes to the process of the Purkinje myocyte communicating with a ventricular cardiac muscle cell in cardiac conduction. Encompasses interactions such as signaling or attachment between one cell and another cell, between a cell and an extracellular matrix, or between a cell and any other aspect of its environment. Sources: GOC:BHF, GOC:mtg_cardiac_conduct_nov11 Relationships: is a type of GO:0086065 Subtypes: Purkinje myocyte to ventricular cardiac muscle cell signaling [GO:0086029], GO:0086055